RNA modification guide activity [GO:0030555] (molecular function) Definition: Specifies the site of a posttranscriptional modification in an RNA molecule by base pairing with a short sequence around the target residue. References: PMID:12457565 Sources: GOC:mah Note: Note that this term describes the activity of a nucleic acid, usually RNA, gene product that interacts with other RNA molecules via base pairing; it should not be used to annotate proteins. Relationships: is a type of RNA binding [GO:0003723] Subtypes: rRNA modification guide activity [GO:0030556], GO:0030557, RNA pseudouridylation guide activity [GO:0030558], GO:0030561, GO:0030566